positive regulation of antifungal peptide biosynthetic process [GO:0006967] (biological process) Relationships: is_a GO:0002804; is a type of GO:0002807; is a type of regulation of antifungal peptide biosynthetic process [GO:0002810]; positively regulates antifungal peptide biosynthetic process [GO:0002783] Definition: Any process that activates or increases the frequency, rate, or extent of antifungal peptide biosynthesis. Also known as: antifungal peptide induction, antifungal polypeptide induction, up regulation of antifungal peptide biosynthetic process, up-regulation of antifungal peptide biosynthetic process, upregulation of antifungal peptide biosynthetic process, activation of antifungal peptide biosynthetic process, stimulation of antifungal peptide biosynthetic process Sources: GOC:mah